{
  "term_id": "UNKNOWN:0003",
  "gene": "UniProtKB:Q6ZV77",
  "term_label": "Unknown cellular component",
  "gene_symbol": "LINC02908",
  "gene_name": "Putative uncharacterized protein LINC02908"
}